{
  "gene": "UniProtKB:X6R8D5",
  "gene_name": "Putative uncharacterized protein GUCA1ANB",
  "gene_symbol": "GUCA1ANB",
  "term_label": "Unknown biological process",
  "term_id": "UNKNOWN:0002"
}